mitotic spindle formation (spindle phase two) [GO:0140641] (biological process) References: PMID:32723864 Definition: The spindle organization process in which the spindle is maintained at a constant length during mitotic metaphase. Also known as: metaphase spindle stability, metaphase spindle stabilization Relationships: is_a mitotic spindle assembly [GO:0090307]